{
  "gene_symbol": "NCBP1",
  "term_label": "nuclear-transcribed mRNA catabolic process, nonsense-mediated decay",
  "term_id": "GO:0000184",
  "gene": "UniProtKB:Q09161",
  "gene_name": "Nuclear cap-binding protein subunit 1"
}